{
  "gene_symbol": "CYP2D6",
  "gene": "UniProtKB:P10635",
  "term_label": "arachidonate metabolic process",
  "gene_name": "Cytochrome P450 2D6",
  "term_id": "GO:0019369"
}